{
  "term_id": "GO:0005829",
  "gene_name": "Heat shock 70 kDa protein 1-like",
  "term_label": "cytosol",
  "gene_symbol": "HSPA1L",
  "gene": "UniProtKB:P34931"
}